{
  "term_label": "cytoplasm",
  "gene_symbol": "CYP2C19",
  "term_id": "GO:0005737",
  "gene_name": "Cytochrome P450 2C19",
  "gene": "UniProtKB:P33261"
}